{
  "gene_symbol": "TRIM7",
  "term_id": "GO:0045087",
  "gene_name": "E3 ubiquitin-protein ligase TRIM7",
  "term_label": "innate immune response",
  "gene": "UniProtKB:Q9C029"
}